{
  "gene_name": "Putative ankyrin repeat domain-containing protein 19",
  "gene_symbol": "ANKRD19P",
  "gene": "UniProtKB:Q9H560",
  "term_id": "UNKNOWN:0001",
  "term_label": "Unknown molecular function"
}